{
  "gene": "UniProtKB:P0CL80",
  "gene_symbol": "GAGE12F",
  "term_label": "Unknown biological process",
  "gene_name": "G antigen 12F",
  "term_id": "UNKNOWN:0002"
}